{
  "gene_name": "Nucleosome assembly protein 1-like 5",
  "term_label": "Unknown biological process",
  "gene_symbol": "NAP1L5",
  "term_id": "UNKNOWN:0002",
  "gene": "UniProtKB:Q96NT1"
}